snRNA-activating protein complex [GO:0019185] (cellular component) Relationships: is a type of transcription regulator complex [GO:0005667] Also known as: SNAPc References: PMID:7715707, PMID:9003788 Definition: A protein complex that recognizes the proximal sequence element of RNA polymerase II and III snRNA promoters.